host multivesicular body [GO:0072494] (CC) Also known as: host cell multivesicular body Definition: A late endosome in which regions of the limiting host cell endosomal membrane invaginate to form internal vesicles; host membrane proteins that enter the internal vesicles are sequestered from the host cytoplasm. Relationships: is a type of GO:0044184 Sources: GOC:rph